{
  "gene_symbol": "ALPI",
  "term_id": "GO:0004035",
  "gene_name": "Intestinal-type alkaline phosphatase",
  "term_label": "alkaline phosphatase activity",
  "gene": "UniProtKB:P09923"
}